{
  "gene": "UniProtKB:Q8NBB4",
  "term_label": "Unknown cellular component",
  "gene_symbol": "ZSCAN1",
  "gene_name": "Zinc finger and SCAN domain-containing protein 1",
  "term_id": "UNKNOWN:0003"
}